N-terminal protein lipidation [GO:0006498] (biological process) Sources: GOC:jl Definition: The covalent attachment of a lipid group to the amino terminus of a protein. Relationships: is a type of GO:0006497; is a type of N-terminal protein amino acid modification [GO:0031365] Subtypes: N-terminal protein myristoylation [GO:0006499], N-terminal protein palmitoylation [GO:0006500]